{
  "term_id": "GO:0006805",
  "gene": "UniProtKB:P05181",
  "term_label": "xenobiotic metabolic process",
  "gene_symbol": "CYP2E1",
  "gene_name": "Cytochrome P450 2E1"
}